{
  "term_id": "GO:0001653",
  "gene_name": "Guanylyl cyclase C",
  "gene": "UniProtKB:P25092",
  "gene_symbol": "GUCY2C",
  "term_label": "peptide receptor activity"
}